melanocyte proliferation [GO:0097325] (BP) Relationships: is a type of epithelial cell proliferation [GO:0050673] Definition: The multiplication or reproduction of melanocytes, resulting in the expansion of a cell population. A melanocyte is a pigment cell derived from the neural crest. It contains melanin-filled pigment granules, which give a brown to black appearance. References: PMID:22637532 Sources: CL:0000148, GOC:uh